pectinesterase inhibitor activity [GO:0046910] (molecular function) Definition: Binds to and stops, prevents or reduces the activity of pectinesterase. Note: See also the molecular function term 'pectinesterase activity ; GO:0030599'. Relationships: is a type of enzyme inhibitor activity [GO:0004857]; negatively regulates GO:0030599 References: PMID:10880981 Sources: GOC:ai